{
  "gene": "UniProtKB:Q86UD1",
  "gene_symbol": "OAF",
  "term_label": "Unknown molecular function",
  "term_id": "UNKNOWN:0001",
  "gene_name": "Out at first protein homolog"
}